{
  "term_id": "GO:0043687",
  "gene": "UniProtKB:P46977",
  "gene_symbol": "STT3A",
  "gene_name": "Dolichyl-diphosphooligosaccharide--protein glycosyltransferase subunit STT3A",
  "term_label": "post-translational protein modification"
}